{
  "term_id": "GO:0005634",
  "term_label": "nucleus",
  "gene_name": "Homeobox protein MSX-1",
  "gene": "UniProtKB:P28360",
  "gene_symbol": "MSX1"
}